{
  "term_label": "Unknown molecular function",
  "gene": "UniProtKB:Q7Z5S9",
  "gene_symbol": "TMEM144",
  "term_id": "UNKNOWN:0001",
  "gene_name": "Transmembrane protein 144"
}